xanthone-containing compound biosynthetic process [GO:2001307] (biological process) Also known as: xanthone-containing compound anabolism, xanthone-containing compound biosynthesis, xanthone-containing compound formation, xanthone-containing compound synthesis, xanthones anabolism, xanthones biosynthesis, xanthones biosynthetic process, xanthones formation, xanthones synthesis, xanthone biosynthesis, xanthone biosynthetic process Relationships: is a type of ketone biosynthetic process [GO:0042181] Sources: GOC:di Regulation: regulated by regulation of xanthone-containing compound biosynthetic process [GO:1900183]; RO_0002212 by negative regulation of xanthone-containing compound biosynthetic process [GO:1900184]; positively regulated by positive regulation of xanthone-containing compound biosynthetic process [GO:1900185] Definition: The chemical reactions and pathways resulting in the formation of a xanthone-containing compound. Subtypes: emericellin biosynthetic process [GO:1900766]